{
  "gene_name": "Ataxin-3",
  "term_id": "GO:0004843",
  "term_label": "cysteine-type deubiquitinase activity",
  "gene": "UniProtKB:P54252",
  "gene_symbol": "ATXN3"
}